{
  "term_id": "GO:0006457",
  "gene_name": "Protein disulfide-isomerase A3",
  "term_label": "protein folding",
  "gene": "UniProtKB:P30101",
  "gene_symbol": "PDIA3"
}